methionyl-tRNA aminoacylation [GO:0006431] (biological process) Relationships: is a type of tRNA aminoacylation for protein translation [GO:0006418] Definition: The process of coupling methionine to methionyl-tRNA, catalyzed by methionyl-tRNA synthetase. The methionyl-tRNA synthetase is a class-I synthetase. The activated amino acid is transferred to the 2'-OH group of a methionine-accetping tRNA. The 2'-O-aminoacyl-tRNA will ultimately migrate to the 3' position via transesterification. Sources: GOC:mcc, ISBN:0716730510 Subtypes: mitochondrial methionyl-tRNA aminoacylation [GO:0070155]